{
  "gene": "UniProtKB:P59538",
  "term_label": "bitter taste receptor activity",
  "gene_name": "Taste receptor type 2 member 31",
  "gene_symbol": "TAS2R31",
  "term_id": "GO:0033038"
}